granulocyte chemotaxis [GO:0071621] (biological process) Subtypes: basophil chemotaxis [GO:0002575], GO:0030593, GO:0048245 Relationships: is a type of GO:0030595; is a type of granulocyte migration [GO:0097530] Sources: GOC:rph Definition: The movement of a granulocyte in response to an external stimulus. Regulation: regulated by regulation of granulocyte chemotaxis [GO:0071622]; negatively regulated by negative regulation of granulocyte chemotaxis [GO:0071623]; positively regulated by positive regulation of granulocyte chemotaxis [GO:0071624]